{
  "term_id": "UNKNOWN:0002",
  "term_label": "Unknown biological process",
  "gene": "UniProtKB:O15442",
  "gene_name": "Metallophosphoesterase domain-containing protein 1",
  "gene_symbol": "MPPED1"
}